{
  "term_label": "Unknown biological process",
  "gene_symbol": "POTEB2",
  "gene_name": "POTE ankyrin domain family member B2",
  "term_id": "UNKNOWN:0002",
  "gene": "UniProtKB:H3BUK9"
}